regulation of cartilage condensation [GO:1902026] (biological process) Subtypes: positive regulation of cartilage condensation [GO:1902027], negative regulation of cartilage condensation [GO:1904932] Relationships: is a type of GO:0050794; regulates cartilage condensation [GO:0001502] References: PMID:17202865 Sources: GOC:TermGenie Definition: Any process that modulates the frequency, rate or extent of cartilage condensation.